{
  "gene_symbol": "RHBDD3",
  "gene": "UniProtKB:Q9Y3P4",
  "term_label": "Unknown cellular component",
  "term_id": "UNKNOWN:0003",
  "gene_name": "Rhomboid domain-containing protein 3"
}